{
  "term_id": "GO:0061630",
  "term_label": "ubiquitin protein ligase activity",
  "gene_symbol": "ZNF598",
  "gene_name": "E3 ubiquitin-protein ligase ZNF598",
  "gene": "UniProtKB:Q86UK7"
}